glycosylceramide catabolic process [GO:0046477] (biological process) Also known as: glycosylceramide breakdown, glycosylceramide catabolism, glycosylceramide degradation Subtypes: glucosylceramide catabolic process [GO:0006680], galactosylceramide catabolic process [GO:0006683] Definition: The chemical reactions and pathways resulting in the breakdown of glycosylceramides, any compound formed by the replacement of the glycosidic hydroxyl group of a cyclic form of a monosaccharide (or derivative) by a ceramide group. Sources: GOC:ai Relationships: is a type of glycosylceramide metabolic process [GO:0006677]; is a type of glycosphingolipid catabolic process [GO:0046479]; is a type of GO:0046514